{
  "gene": "UniProtKB:Q9Y5F7",
  "term_id": "GO:0005886",
  "term_label": "plasma membrane",
  "gene_symbol": "PCDHGC4",
  "gene_name": "Protocadherin gamma-C4"
}